nucleotide-sulfate transmembrane transporter activity [GO:0005340] (molecular function) Definition: Enables the transfer of nucleotide-sulfate from one side of a membrane to the other. Sources: GOC:mtg_transport Relationships: is a type of GO:0015116; is a type of organophosphate ester transmembrane transporter activity [GO:0015605]; is a type of nucleobase-containing compound transmembrane transporter activity [GO:0015932] Also known as: nucleotide-sulphate transporter activity